{
  "gene_name": "Centromere protein X",
  "term_label": "FANCM-MHF complex",
  "gene": "UniProtKB:A8MT69",
  "gene_symbol": "CENPX",
  "term_id": "GO:0071821"
}